{
  "gene": "UniProtKB:P35228",
  "gene_name": "Nitric oxide synthase, inducible",
  "term_id": "GO:0009725",
  "gene_symbol": "NOS2",
  "term_label": "response to hormone"
}